{
  "gene_symbol": "VPS37D",
  "gene_name": "Vacuolar protein sorting-associated protein 37D",
  "term_id": "GO:0000813",
  "gene": "UniProtKB:Q86XT2",
  "term_label": "ESCRT I complex"
}